{
  "gene_symbol": "SLC6A3",
  "term_label": "Unknown molecular function",
  "gene_name": "Sodium-dependent dopamine transporter",
  "gene": "UniProtKB:Q01959",
  "term_id": "UNKNOWN:0001"
}